{
  "gene_symbol": "CCDC28A-AS1",
  "gene": "UniProtKB:A0A096LPI5",
  "gene_name": "Putative uncharacterized protein CCDC28A-AS1",
  "term_id": "UNKNOWN:0002",
  "term_label": "Unknown biological process"
}